free sarcoplasmic reticulum membrane [GO:0014702] (cellular component) Relationships: is a type of sarcoplasmic reticulum membrane [GO:0033017] Definition: The part of the sarcoplasmic reticulum membrane that contains calcium pumps and is devoted to calcium uptake. The free sarcoplasmic reticulum membrane consists of the longitudinal sarcoplasmic reticulum membrane and the non-junctional region of the terminal cisterna membrane. Sources: GOC:mtg_muscle